{
  "term_id": "GO:0008284",
  "gene": "UniProtKB:P05019",
  "term_label": "positive regulation of cell population proliferation",
  "gene_symbol": "IGF1",
  "gene_name": "Insulin-like growth factor I"
}